{
  "term_label": "extracellular space",
  "gene_name": "Interferon alpha-4",
  "gene": "UniProtKB:P05014",
  "term_id": "GO:0005615",
  "gene_symbol": "IFNA4"
}